formation of infection structure [GO:0075015] (biological process) Definition: The formation of a symbiont structure that serves to infect its host organism. It includes physiological, developmental, and morphological changes of the symbiont. The host is defined as the larger of the organisms involved in a symbiotic interaction. Subtypes: appressorium formation [GO:0075016], formation of appressorium germ tube hook structure [GO:0075029], penetration peg formation [GO:0075053], infection cushion formation [GO:0075183], hyphopodium formation [GO:0075187], haustorium mother cell formation [GO:0075192], haustorium neck formation [GO:0075197], GO:0075201 Note: Note that this term should not be used to annotate gene products of the host. It should only be used to annotate those gene products of the symbiont involved in this process. Sources: GOC:pamgo_curators Relationships: is a type of anatomical structure formation involved in morphogenesis [GO:0048646]; is part of symbiont entry into host [GO:0044409] Also known as: formation of host infection structure, formation by symbiont of infection structure on or near host, formation of host penetration structure, formation of infection structure on or near host